{
  "term_id": "GO:0032039",
  "gene": "UniProtKB:Q96CB8",
  "gene_name": "Integrator complex subunit 12",
  "gene_symbol": "INTS12",
  "term_label": "integrator complex"
}